negative regulation of heterotypic cell-cell adhesion [GO:0034115] (biological process) Subtypes: negative regulation of platelet rolling [GO:0160019] Sources: GOC:add Relationships: is_a GO:0022408; is a type of regulation of heterotypic cell-cell adhesion [GO:0034114]; is a type of regulation of cell-cell adhesion involved in gastrulation [GO:0070587]; negatively regulates heterotypic cell-cell adhesion [GO:0034113] Definition: Any process that stops, prevents, or reduces the frequency, rate, or extent of heterotypic cell-cell adhesion.